{
  "term_id": "GO:0003810",
  "term_label": "protein-glutamine gamma-glutamyltransferase activity",
  "gene_name": "Protein-glutamine gamma-glutamyltransferase 5",
  "gene_symbol": "TGM5",
  "gene": "UniProtKB:O43548"
}